positive regulation of establishment of bipolar cell polarity regulating cell shape [GO:0061161] (biological process) Definition: Any process that increases the rate, frequency or extent of the establishment of bipolar cell polarity that regulates the shape of a cell. Relationships: is a type of regulation of establishment of bipolar cell polarity regulating cell shape [GO:0061160]; is_a GO:0061173; is a type of positive regulation of establishment or maintenance of bipolar cell polarity regulating cell shape [GO:2000247] Sources: GOC:dph, GOC:vw